L-lysine N6-acetyltransferase [GO:0090595] (molecular function) Also known as: acetyl-CoA:L-lysine N6-acetyltransferase Relationships: is a type of L-amino-acid N-acetyltransferase activity [GO:0140085] Sources: RHEA:69476 Definition: Catalysis of the reaction: acetyl-CoA + L-lysine = CoA + H+ + N(6)-acetyl-L-lysine.